{
  "term_id": "GO:0046327",
  "term_label": "glycerol biosynthetic process from pyruvate",
  "gene_name": "Phosphoenolpyruvate carboxykinase, cytosolic [GTP]",
  "gene": "UniProtKB:P35558",
  "gene_symbol": "PCK1"
}